{
  "gene": "UniProtKB:Q9NY91",
  "term_label": "transmembrane transporter activity",
  "gene_name": "Probable glucose sensor protein SLC5A4",
  "term_id": "GO:0022857",
  "gene_symbol": "SLC5A4"
}